{
  "gene": "UniProtKB:P30050",
  "term_label": "translation",
  "term_id": "GO:0006412",
  "gene_symbol": "RPL12",
  "gene_name": "Large ribosomal subunit protein uL11"
}